{
  "term_id": "GO:0051123",
  "gene_symbol": "TAF11L7",
  "term_label": "RNA polymerase II preinitiation complex assembly",
  "gene_name": "TATA-box-binding protein-associated factor 11-like protein 7",
  "gene": "UniProtKB:P0DW12"
}